ubiquitin activating enzyme activity [GO:0004839] (molecular function) Note: The ubiquitin activating enzyme catalyzes a ligation reaction. Definition: Catalysis of the reaction: E1 + ubiquitin + ATP--> E1-ubiquitin + AMP + PPi, where the E1-ubiquitin linkage is a thioester bond between the C-terminal glycine of Ub and a sulfhydryl side group of an E1 cysteine residue. This is the first step in a cascade of reactions in which ubiquitin is ultimately added to a protein substrate. Relationships: is a type of GO:0008641; is part of protein ubiquitination [GO:0016567] Sources: GOC:BioGRID, Wikipedia:Ubiquitin-activating_enzyme Also known as: E1 ubiquitin-activating enzyme